response to estrogen [GO:0043627] (BP) Subtypes: cellular response to estrogen stimulus [GO:0071391] Also known as: response to estrogen stimulus, response to oestrogen stimulus, response to 17alpha-ethynylestradiol Relationships: is_a response to hormone [GO:0009725] Definition: Any process that results in a change in state or activity of a cell or an organism (in terms of movement, secretion, enzyme production, gene expression, etc.) as a result of stimulus by an estrogen, C18 steroid hormones that can stimulate the development of female sexual characteristics. Sources: GOC:jl, ISBN:0198506732